indoleacetic acid conjugate metabolic process [GO:0033473] (biological process) Relationships: is a type of indole-containing compound metabolic process [GO:0042430] Also known as: IAA conjugate metabolic process, indole acetic acid conjugate metabolic process, indole acetic acid conjugate metabolism, indoleacetic acid conjugate metabolism Sources: GOC:mah Definition: The chemical reactions and pathways involving any indole-3-acetic acid conjugate, a form of indoleacetic acid covalently bound to another molecule. Subtypes: GO:0033474